{
  "term_label": "Unknown cellular component",
  "term_id": "UNKNOWN:0003",
  "gene": "UniProtKB:Q9UBG3",
  "gene_symbol": "CRNN",
  "gene_name": "Cornulin"
}